apical constriction [GO:0003383] (BP) Definition: The actin-mediated process that results in the contraction of the apical end of a polarized columnar epithelial cell. Subtypes: apical constriction involved in gastrulation [GO:0003384] Relationships: is a type of actin-mediated cell contraction [GO:0070252]; is part of epithelial cell morphogenesis [GO:0003382] Sources: GOC:ascb_2009, GOC:dph, GOC:tb